{
  "gene_name": "Frizzled-4",
  "gene_symbol": "FZD4",
  "term_label": "Wnt-protein binding",
  "term_id": "GO:0017147",
  "gene": "UniProtKB:Q9ULV1"
}